SET domain binding [GO:0070984] (molecular function) Definition: Binding to a SET domain of a protein. SET domains are named after three Drosophila proteins that contain this domain: Su(var), E(z) and trithorax. SET domains are associated with histone lysine methylation. References: PMID:12575990 Sources: GOC:sart, Pfam:PF00856 Also known as: SET binding Relationships: is a type of protein domain specific binding [GO:0019904]